{
  "gene_symbol": "MAPK1",
  "gene_name": "Mitogen-activated protein kinase 1",
  "term_id": "GO:0004674",
  "gene": "UniProtKB:P28482",
  "term_label": "protein serine/threonine kinase activity"
}